{
  "term_label": "cilium assembly",
  "gene_name": "Cilia- and flagella-associated protein 161",
  "term_id": "GO:0060271",
  "gene_symbol": "CFAP161",
  "gene": "UniProtKB:Q6P656"
}